{
  "gene_symbol": "IGFL3",
  "gene": "UniProtKB:Q6UXB1",
  "term_label": "signaling receptor binding",
  "term_id": "GO:0005102",
  "gene_name": "Insulin growth factor-like family member 3"
}